negative regulation of phosphate metabolic process [GO:0045936] (biological process) Sources: GOC:go_curators Subtypes: negative regulation of inositol phosphate biosynthetic process [GO:0010920], negative regulation of dephosphorylation [GO:0035305], negative regulation of phosphorylation [GO:0042326], negative regulation of nucleotide metabolic process [GO:0045980], negative regulation of thiamine diphosphate biosynthetic process [GO:0070617], negative regulation of UDP-N-acetylglucosamine biosynthetic process [GO:0106279], GO:0160218, negative regulation of butyryl-CoA biosynthetic process from acetyl-CoA [GO:1900495], negative regulation of butyryl-CoA catabolic process to butanol [GO:1900498], negative regulation of butyryl-CoA catabolic process to butyrate [GO:1900501], GO:1900972, negative regulation of tetrapyrrole biosynthetic process from glycine and succinyl-CoA [GO:1901414], GO:1903726 Relationships: is a type of negative regulation of phosphorus metabolic process [GO:0010563]; negatively regulates phosphate-containing compound metabolic process [GO:0006796] Also known as: down regulation of phosphate metabolic process, down-regulation of phosphate metabolic process, downregulation of phosphate metabolic process, negative regulation of phosphate metabolism, inhibition of phosphate metabolic process Definition: Any process that stops, prevents, or reduces the frequency, rate or extent of the chemical reactions and pathways involving phosphates.